rRNA base methylation [GO:0070475] (BP) Definition: The addition of a methyl group to an atom in the nucleoside base portion of a nucleotide residue in an rRNA molecule. Relationships: is a type of GO:0031167 Subtypes: rRNA (guanine-N7)-methylation [GO:0070476] Sources: GOC:mah